mating pheromone secretion involved in positive regulation of conjugation with cellular fusion [GO:0071631] (biological process) Definition: The regulated release of a mating pheromone, a peptide hormone that induces a behavioral or physiological response(s) from a responding organism or cell, that positively regulates a conjugation process that results in the union of cellular and genetic information from compatible mating types. Sources: GOC:elh, GOC:jh, GOC:mah Also known as: mating-type pheromone secretion involved in conjugation with cellular fusion, peptide pheromone export involved in positive regulation of conjugation with cellular fusion Relationships: is a type of GO:0031139; is a type of mating pheromone secretion [GO:0071834]